noradrenergic synapse [GO:0098692] (cellular component) Relationships: is a type of synapse [GO:0045202] Sources: GOC:dos Definition: A synapse that uses noradrenaline as a neurotransmitter.